{
  "term_id": "GO:0009617",
  "gene_name": "T cell receptor alpha variable 24",
  "term_label": "response to bacterium",
  "gene": "UniProtKB:A0A0B4J272",
  "gene_symbol": "TRAV24"
}